{
  "term_id": "GO:0045944",
  "term_label": "positive regulation of transcription by RNA polymerase II",
  "gene_symbol": "MTF1",
  "gene_name": "Metal regulatory transcription factor 1",
  "gene": "UniProtKB:Q14872"
}